regulation of synaptic plasticity by chemical substance [GO:0051913] (biological process) Also known as: regulation of synaptic plasticity by drug Definition: The process in which a chemical substance modulates synaptic plasticity, the ability of synapses to change as circumstances require. Relationships: is a type of GO:0048167; is part of response to chemical [GO:0042221] Subtypes: positive regulation of synaptic plasticity by chemical substance [GO:0051914] Sources: GOC:ai